{
  "gene": "UniProtKB:Q9BT25",
  "gene_name": "HAUS augmin-like complex subunit 8",
  "term_id": "GO:0005880",
  "term_label": "nuclear microtubule",
  "gene_symbol": "HAUS8"
}